indoleacetamide hydrolase activity [GO:0043864] (molecular function) Also known as: IAH, indole acetamide hydrolase activity, indole-3-acetamide hydrolase activity, IaaH, Tms2 Sources: GOC:jl, RHEA:34371 Definition: Catalysis of the reaction: iH2O + indole-3-acetamide = (indol-3-yl)acetate + NH4+. Indole-3-acetamide is known as IAM and indole-3-acetate as IAA. Relationships: is a type of amidase activity [GO:0004040]